{
  "term_label": "intracellular zinc ion homeostasis",
  "gene_symbol": "SLC30A5",
  "gene_name": "Proton-coupled zinc antiporter SLC30A5",
  "term_id": "GO:0006882",
  "gene": "UniProtKB:Q8TAD4"
}